{
  "term_label": "positive regulation of transcription by RNA polymerase II",
  "gene_symbol": "NR1H4",
  "term_id": "GO:0045944",
  "gene_name": "Bile acid receptor",
  "gene": "UniProtKB:Q96RI1"
}